{
  "term_label": "nucleus",
  "gene": "UniProtKB:A6NCW0",
  "gene_name": "Ubiquitin carboxyl-terminal hydrolase 17-like protein 3",
  "gene_symbol": "USP17L3",
  "term_id": "GO:0005634"
}